regulation of acyl-CoA biosynthetic process [GO:0050812] (biological process) Subtypes: GO:0010510, regulation of butyryl-CoA biosynthetic process from acetyl-CoA [GO:1900494] Definition: Any process that modulates the frequency, rate or extent of the chemical reactions and pathways resulting in the formation of acyl-CoA. Relationships: is a type of GO:0009889; is a type of GO:0019217; is a type of regulation of nucleobase-containing compound metabolic process [GO:0019219]; is a type of regulation of amide metabolic process [GO:0034248]; is a type of regulation of sulfur metabolic process [GO:0042762]; is a type of regulation of phosphorus metabolic process [GO:0051174]; regulates acyl-CoA biosynthetic process [GO:0071616] Sources: GOC:ai Also known as: regulation of acyl-CoA anabolism, regulation of acyl-CoA biosynthesis, regulation of acyl-CoA formation, regulation of acyl-CoA synthesis